presynaptic active zone disassembly [GO:1904072] (biological process) Relationships: is a type of cellular component disassembly [GO:0022411]; is a type of presynaptic active zone organization [GO:1990709] Sources: GOC:TermGenie, GOC:pr, GO_REF:0000079, ISBN:9780387325606 Definition: The disaggregation of a presynaptic active zone into its constituent components. Also known as: pre-synaptic active zone disassembly, pre-synaptic active zone component disassembly